AV node cell action potential [GO:0086016] (biological process) Also known as: AV node cardiac muscle cell action potential, atrioventricular node cardiac muscle cell action potential Definition: An action potential that occurs in an atrioventricular node cardiac muscle cell. Relationships: is a type of cardiac muscle cell action potential [GO:0086001]; is part of AV node cell to bundle of His cell signaling [GO:0086027] Sources: GOC:BHF, GOC:mtg_cardiac_conduct_nov11 Regulation: regulated by regulation of AV node cell action potential [GO:0098904]; RO_0002212 by negative regulation of AV node cell action potential [GO:1903950]; positively regulated by positive regulation of AV node cell action potential [GO:1903951]